protein localization to plasma membrane raft [GO:0044860] (biological process) Sources: GOC:jl Subtypes: protein transport into plasma membrane raft [GO:0044861] Definition: A process in which a protein is transported to, or maintained in, a location within a plasma membrane raft. Relationships: is a type of protein localization to membrane raft [GO:1903044]; is a type of protein localization to cell periphery [GO:1990778]